{
  "gene_name": "Zinc transporter 7",
  "gene_symbol": "SLC30A7",
  "gene": "UniProtKB:Q8NEW0",
  "term_id": "GO:0031410",
  "term_label": "cytoplasmic vesicle"
}